{
  "gene_name": "Calcium-binding and coiled-coil domain-containing protein 1",
  "gene": "UniProtKB:Q9P1Z2",
  "term_label": "positive regulation of transcription by RNA polymerase II",
  "gene_symbol": "CALCOCO1",
  "term_id": "GO:0045944"
}